{
  "gene_symbol": "CIRBP",
  "gene": "UniProtKB:Q14011",
  "term_label": "mRNA splicing, via spliceosome",
  "gene_name": "Cold-inducible RNA-binding protein",
  "term_id": "GO:0000398"
}